alpha-linolenic acid metabolic process [GO:0036109] (biological process) Relationships: is a type of long-chain fatty acid metabolic process [GO:0001676]; is a type of unsaturated fatty acid metabolic process [GO:0033559]; is_a olefinic compound metabolic process [GO:0120254] References: PMID:15538555 Definition: The chemical reactions and pathways involving alpha-linolenic acid, an unsaturated omega-6 fatty acid that has the molecular formula C18H32O2. Also known as: ALA metabolism, alpha-linolenic acid metabolism